{
  "term_label": "G protein-coupled receptor signaling pathway",
  "gene_name": "Vasopressin V2 receptor",
  "gene": "UniProtKB:P30518",
  "term_id": "GO:0007186",
  "gene_symbol": "AVPR2"
}